negative regulation of hepatocyte differentiation [GO:0070367] (biological process) Also known as: down regulation of hepatocyte differentiation, down-regulation of hepatocyte differentiation, downregulation of hepatocyte differentiation, negative regulation of liver cell differentiation, inhibition of hepatocyte differentiation Sources: GOC:mah, GOC:sl Relationships: is a type of negative regulation of epithelial cell differentiation [GO:0030857]; is a type of negative regulation of multicellular organismal process [GO:0051241]; is a type of regulation of hepatocyte differentiation [GO:0070366]; negatively regulates hepatocyte differentiation [GO:0070365] Definition: Any process that stops or decreases the rate or extent of hepatocyte differentiation.